{
  "gene_name": "NEDD4 family-interacting protein 1",
  "gene": "UniProtKB:Q9BT67",
  "gene_symbol": "NDFIP1",
  "term_label": "endoplasmic reticulum",
  "term_id": "GO:0005783"
}